{
  "gene_name": "Voltage-dependent calcium channel gamma-4 subunit",
  "gene": "UniProtKB:Q9UBN1",
  "term_id": "GO:0098970",
  "gene_symbol": "CACNG4",
  "term_label": "postsynaptic neurotransmitter receptor diffusion trapping"
}